androgen catabolic process [GO:0006710] (biological process) Also known as: androgen breakdown, androgen catabolism, androgen degradation Definition: The chemical reactions and pathways resulting in the breakdown of androgens, C19 steroid hormones that can stimulate the development of male sexual characteristics. Sources: ISBN:0198506732 Relationships: is a type of steroid catabolic process [GO:0006706]; is a type of androgen metabolic process [GO:0008209]; is_a hormone catabolic process [GO:0042447]